{
  "gene_symbol": "CALML3",
  "term_label": "calcium ion binding",
  "gene_name": "Calmodulin-like protein 3",
  "term_id": "GO:0005509",
  "gene": "UniProtKB:P27482"
}